{
  "gene": "UniProtKB:P42331",
  "gene_name": "Rho GTPase-activating protein 25",
  "term_id": "GO:0005096",
  "term_label": "GTPase activator activity",
  "gene_symbol": "ARHGAP25"
}